{
  "term_id": "GO:0042147",
  "gene": "UniProtKB:O60499",
  "term_label": "retrograde transport, endosome to Golgi",
  "gene_symbol": "STX10",
  "gene_name": "Syntaxin-10"
}